methane metabolic process [GO:0015947] (biological process) Sources: ISBN:0198506732 Relationships: is a type of GO:0120252 Also known as: methane metabolism Subtypes: methanogenesis [GO:0015948], GO:0046188 Definition: The chemical reactions and pathways involving methane, a colorless, odorless, flammable gas with the formula CH4. It is the simplest of the alkanes.